regulation of mitotic cell cycle spindle assembly checkpoint [GO:0090266] (biological process) Sources: GOC:mtg_cell_cycle Subtypes: GO:0090267, negative regulation of mitotic spindle assembly checkpoint signaling [GO:0140499] Definition: Any process that modulates the rate, frequency, or extent of the mitotic cell cycle spindle assembly checkpoint, a cell cycle checkpoint that delays the metaphase/anaphase transition of a mitotic nuclear division until the spindle is correctly assembled and chromosomes are attached to the spindle. Relationships: is a type of regulation of mitotic nuclear division [GO:0007088]; is a type of regulation of mitotic sister chromatid separation [GO:0010965]; is a type of regulation of mitotic metaphase/anaphase transition [GO:0030071]; is a type of regulation of mitotic sister chromatid segregation [GO:0033047]; is_a regulation of mitotic spindle checkpoint [GO:1903504]; regulates GO:0007094